{
  "gene": "UniProtKB:P81172",
  "gene_name": "Hepcidin",
  "term_id": "GO:0006879",
  "term_label": "intracellular iron ion homeostasis",
  "gene_symbol": "HAMP"
}